{
  "term_id": "UNKNOWN:0001",
  "gene": "UniProtKB:Q9NRY2",
  "gene_name": "SOSS complex subunit C",
  "gene_symbol": "INIP",
  "term_label": "Unknown molecular function"
}